lymphatic endothelial cell migration [GO:1904977] (biological process) Definition: The orderly movement of a lymphatic endothelial cell from one site to another in the wall of a lymphatic vessel. Relationships: is a type of endothelial cell migration [GO:0043542]; is part of lymph vessel morphogenesis [GO:0036303] References: PMID:25745057 Sources: GOC:TermGenie, GO_REF:0000091